norepinephrine:sodium symporter activity [GO:0005334] (molecular function) Relationships: is a type of monoamine transmembrane transporter activity [GO:0008504]; is a type of sodium:chloride symporter activity [GO:0015378]; is part of norepinephrine uptake [GO:0051620] Definition: Enables the transfer of a solute or solutes from one side of a membrane to the other according to the reaction: norepinephrine(out) + Na+(out) + Cl-(out) = norepinephrine(in) + Na+(in) + Cl-(in). Also known as: levarterenol transporter activity, noradrenaline transporter activity, norepinephrine transmembrane transporter activity, norepinephrine:sodium:chloride symporter activity, sodium/norepinephrine symporter activity References: PMID:21752877, PMID:22519513 Sources: TC:2.A.22.1.2